{
  "term_label": "sphingolipid biosynthetic process",
  "gene": "UniProtKB:Q53FV1",
  "term_id": "GO:0030148",
  "gene_name": "ORM1-like protein 2",
  "gene_symbol": "ORMDL2"
}